{
  "term_label": "RNA helicase activity",
  "gene": "UniProtKB:Q13283",
  "term_id": "GO:0003724",
  "gene_symbol": "G3BP1",
  "gene_name": "Ras GTPase-activating protein-binding protein 1"
}